{
  "term_id": "GO:0005634",
  "gene": "UniProtKB:Q8N8Y5",
  "gene_symbol": "ZFP41",
  "gene_name": "Zinc finger protein 41 homolog",
  "term_label": "nucleus"
}